{
  "gene_name": "Cadherin-1",
  "term_id": "GO:0008013",
  "term_label": "beta-catenin binding",
  "gene": "UniProtKB:P12830",
  "gene_symbol": "CDH1"
}